ascopyrone tautomerase activity [GO:0034018] (molecular function) Definition: Catalysis of the reaction: 1,5-anhydro-4-deoxy-D-glycero-hex-3-en-2-ulose = 1,5-anhydro-4-deoxy-D-glycero-hex-1-en-3-ulose. Relationships: is a type of GO:0016862 Also known as: 1,5-anhydro-D-glycero-hex-3-en-2-ulose delta3-delta1-isomerase activity, 1,5-anhydro-D-glycero-hex-3-en-2-ulose tautomerase activity, APM tautomerase activity, APTM, ascopyrone P tautomerase activity, ascopyrone intramolecular oxidoreductase activity, ascopyrone isomerase activity Sources: EC:5.3.2.7